negative regulation of response to wounding [GO:1903035] (biological process) Also known as: down regulation of physiological response to wounding, down regulation of response to wounding, down-regulation of physiological response to wounding, down-regulation of response to wounding, downregulation of physiological response to wounding, downregulation of response to wounding, negative regulation of physiological response to wounding, inhibition of physiological response to wounding, inhibition of response to wounding Subtypes: negative regulation of axon regeneration [GO:0048681], GO:0061045, negative regulation of inflammatory response to wounding [GO:0106015] References: PMID:19164535 Sources: GOC:TermGenie, GOC:kmv, GO_REF:0000058 Relationships: is a type of negative regulation of response to stimulus [GO:0048585]; is a type of regulation of response to wounding [GO:1903034]; negatively regulates response to wounding [GO:0009611] Definition: Any process that stops, prevents or reduces the frequency, rate or extent of response to wounding.